{
  "gene": "UniProtKB:Q9NZJ5",
  "gene_name": "Eukaryotic translation initiation factor 2-alpha kinase 3",
  "term_id": "GO:0006446",
  "gene_symbol": "EIF2AK3",
  "term_label": "regulation of translational initiation"
}